{
  "term_label": "GTPase activity",
  "gene_symbol": "RAB8A",
  "gene": "UniProtKB:P61006",
  "gene_name": "Ras-related protein Rab-8A",
  "term_id": "GO:0003924"
}